mRNA cap methyltransferase RNMT:RAMAC complex [GO:0160130] (CC) Relationships: is a type of GO:0034708 References: PMID:22099306 Definition: A protein complex that consists of RNA guanine-7 methyltransferase (RNMT) and RNA guanine-7 methyltransferase activating subunit (RAMAC) and is involved in mRNA cap methylation.